{
  "term_id": "UNKNOWN:0002",
  "gene_symbol": "IRGC",
  "term_label": "Unknown biological process",
  "gene": "UniProtKB:Q6NXR0",
  "gene_name": "Interferon-inducible GTPase 5"
}